dendritic spine origin [GO:0150004] (CC) Definition: The part of the dendritic spine neck where the spine arises from the dendritic shaft. References: PMID:9030614 Sources: GOC:aruk, GOC:bc Relationships: is a type of cellular anatomical structure [GO:0110165]; is part of GO:0044326